{
  "gene_symbol": "CSHL1",
  "term_id": "GO:0008083",
  "gene_name": "Chorionic somatomammotropin hormone-like 1",
  "gene": "UniProtKB:Q14406",
  "term_label": "growth factor activity"
}